{
  "gene_name": "Alpha-1-acid glycoprotein 2",
  "gene": "UniProtKB:P19652",
  "term_label": "Unknown molecular function",
  "gene_symbol": "ORM2",
  "term_id": "UNKNOWN:0001"
}